{
  "term_id": "UNKNOWN:0003",
  "term_label": "Unknown cellular component",
  "gene": "UniProtKB:Q6ZMQ8",
  "gene_name": "Serine_threonine-protein kinase LMTK1",
  "gene_symbol": "AATK"
}